vacuolar proton-transporting V-type ATPase, V1 domain [GO:0000221] (cellular component) Also known as: vacuolar hydrogen ion-transporting ATPase V1 domain Note: Note that this domain generally consists of eight subunits. Definition: The V1 domain of a proton-transporting V-type ATPase found in the vacuolar membrane. Subtypes: lysosomal proton-transporting V-type ATPase, V1 domain [GO:0046612] References: PMID:16449553 Sources: GOC:mah Relationships: is a type of proton-transporting V-type ATPase, V1 domain [GO:0033180]; is part of GO:0016471